{
  "gene_symbol": "CAV1",
  "term_id": "GO:0001937",
  "term_label": "negative regulation of endothelial cell proliferation",
  "gene_name": "Caveolin-1",
  "gene": "UniProtKB:Q03135"
}